{
  "gene_symbol": "KRTAP10-12",
  "gene_name": "Keratin-associated protein 10-12",
  "term_id": "UNKNOWN:0002",
  "gene": "UniProtKB:P60413",
  "term_label": "Unknown biological process"
}